{
  "term_id": "GO:0015693",
  "term_label": "magnesium ion transport",
  "gene_name": "Magnesium transporter NIPA2",
  "gene": "UniProtKB:Q8N8Q9",
  "gene_symbol": "NIPA2"
}